nicotinamide nucleotide metabolic process [GO:0046496] (biological process) Definition: The chemical reactions and pathways involving nicotinamide nucleotides, any nucleotide that contains combined nicotinamide. Sources: ISBN:0198506732 Also known as: nicotinamide nucleotide metabolism Relationships: is a type of nucleotide metabolic process [GO:0009117]; is a type of GO:0072524 Subtypes: glycolytic process [GO:0006096], NADP+ metabolic process [GO:0006739], nicotinamide nucleotide biosynthetic process [GO:0019359], GO:0019674, sulphoglycolysis [GO:0061722]